{
  "gene_symbol": "GABRB2",
  "gene": "UniProtKB:P47870",
  "gene_name": "Gamma-aminobutyric acid receptor subunit beta-2",
  "term_id": "GO:0051932",
  "term_label": "synaptic transmission, GABAergic"
}